{
  "term_label": "morphogenesis of an epithelium",
  "gene": "UniProtKB:O76011",
  "gene_name": "Keratin, type I cuticular Ha4",
  "gene_symbol": "KRT34",
  "term_id": "GO:0002009"
}